{
  "term_label": "plasma membrane",
  "gene_symbol": "OR2L2",
  "gene": "UniProtKB:Q8NH16",
  "gene_name": "Olfactory receptor 2L2",
  "term_id": "GO:0005886"
}